{
  "gene_symbol": "AHRR",
  "term_label": "nuclear receptor activity",
  "gene": "UniProtKB:A9YTQ3",
  "gene_name": "Aryl hydrocarbon receptor repressor",
  "term_id": "GO:0004879"
}